{
  "term_label": "reticulophagy",
  "gene_symbol": "UFM1",
  "gene_name": "Ubiquitin-fold modifier 1",
  "term_id": "GO:0061709",
  "gene": "UniProtKB:P61960"
}